glucose catabolic process to pyruvate utilizing ADP [GO:0061719] (BP) Definition: The chemical reactions and pathways resulting in the breakdown of glucose into pyruvate, with the concomitant production of a small amount of ATP and the utilization of ADP in the initial kinase reactions. Sources: GOC:dph, MetaCyc:P341-PWY Relationships: is_a generation of precursor metabolites and energy [GO:0006091]; is_a glucose catabolic process to pyruvate [GO:0061718]; has part fructose-bisphosphate aldolase activity [GO:0004332]; has part glucose-6-phosphate isomerase activity [GO:0004347]; BFO_0000051 phosphoglycerate kinase activity [GO:0004618]; has part GO:0004619; has part pyruvate kinase activity [GO:0004743]; has part triose-phosphate isomerase activity [GO:0004807]; has part glyceraldehyde-3-phosphate dehydrogenase (ferredoxin) activity [GO:0043797]; has part GO:0043843; BFO_0000051 ADP-specific phosphofructokinase activity [GO:0043844]